fluorescent chlorophyll catabolite monooxygenase (deformylase) activity [GO:0106371] (molecular function) References: PMID:23723324 Sources: RHEA:67172 Relationships: is a type of oxidoreductase activity, acting on paired donors, with incorporation or reduction of molecular oxygen, NAD(P)H as one donor, and incorporation of one atom of oxygen [GO:0016709] Definition: Catalysis of the reaction: O2 + primary fluorescent chlorophyll catabolite + reduced [NADPH--hemoprotein reductase] = formate + 2 H+ + oxidized [NADPH--hemoprotein reductase] + primary fluorescent dioxobilin-type chlorophyll catabolite.